{
  "gene": "UniProtKB:Q9P003",
  "gene_symbol": "CNIH4",
  "gene_name": "Protein cornichon homolog 4",
  "term_id": "GO:0030134",
  "term_label": "COPII-coated ER to Golgi transport vesicle"
}